{
  "gene_name": "NACHT, LRR and PYD domains-containing protein 12",
  "gene_symbol": "NLRP12",
  "term_label": "positive regulation of MHC class I biosynthetic process",
  "gene": "UniProtKB:P59046",
  "term_id": "GO:0045345"
}